{
  "gene_symbol": "IL13RA1",
  "gene_name": "Interleukin-13 receptor subunit alpha-1",
  "gene": "UniProtKB:P78552",
  "term_label": "external side of plasma membrane",
  "term_id": "GO:0009897"
}